{
  "gene": "UniProtKB:O94856",
  "gene_name": "Neurofascin",
  "gene_symbol": "NFASC",
  "term_label": "cell-cell adhesion mediator activity",
  "term_id": "GO:0098632"
}